{
  "term_id": "GO:0030036",
  "gene_symbol": "FMN1",
  "gene_name": "Formin-1",
  "term_label": "actin cytoskeleton organization",
  "gene": "UniProtKB:Q68DA7"
}